{
  "gene_name": "Uncharacterized protein C1orf87",
  "gene_symbol": "C1orf87",
  "term_label": "Unknown biological process",
  "term_id": "UNKNOWN:0002",
  "gene": "UniProtKB:Q8N0U7"
}